{
  "gene": "UniProtKB:Q96SZ4",
  "term_id": "GO:0006357",
  "gene_symbol": "ZSCAN10",
  "gene_name": "Zinc finger and SCAN domain-containing protein 10",
  "term_label": "regulation of transcription by RNA polymerase II"
}